regulation of response to benzene [GO:1901451] (BP) Relationships: is a type of GO:0048583; regulates response to benzene [GO:1901423] Definition: Any process that modulates the frequency, rate or extent of response to benzene. Subtypes: GO:1901452, positive regulation of response to benzene [GO:1901453] Sources: GOC:TermGenie, GOC:mengo_curators